isotype switching to IgG isotypes [GO:0048291] (BP) Also known as: class switching to IgG isotypes, isotype switch recombination to IgG isotypes References: PMID:12370374, PMID:2113175, PMID:9186655 Sources: ISBN:0781735149 Definition: The switching of activated B cells from IgM biosynthesis to biosynthesis of an IgG isotype, accomplished through a recombination process involving an intrachromosomal deletion between switch regions that reside 5' of the IgM and one of the IgG constant region gene segments in the immunoglobulin heavy chain locus. Regulation: regulated by regulation of isotype switching to IgG isotypes [GO:0048302]; negatively regulated by negative regulation of isotype switching to IgG isotypes [GO:0048303]; positively regulated by positive regulation of isotype switching to IgG isotypes [GO:0048304] Relationships: is a type of GO:0045190